{
  "term_label": "protein K11-linked ubiquitination",
  "gene_symbol": "ANAPC1",
  "gene": "UniProtKB:Q9H1A4",
  "gene_name": "Anaphase-promoting complex subunit 1",
  "term_id": "GO:0070979"
}